{
  "gene_name": "ER membrane protein complex subunit 10",
  "term_id": "UNKNOWN:0002",
  "gene": "UniProtKB:Q5UCC4",
  "gene_symbol": "EMC10",
  "term_label": "Unknown biological process"
}